{
  "term_id": "UNKNOWN:0001",
  "gene_symbol": "DRC7",
  "term_label": "Unknown molecular function",
  "gene_name": "Dynein regulatory complex subunit 7",
  "gene": "UniProtKB:Q8IY82"
}